{
  "term_label": "nucleoplasm",
  "gene_symbol": "NUFIP2",
  "gene_name": "FMR1-interacting protein NUFIP2",
  "term_id": "GO:0005654",
  "gene": "UniProtKB:Q7Z417"
}